{
  "term_label": "DNA-binding transcription factor activity, RNA polymerase II-specific",
  "gene": "UniProtKB:O43186",
  "term_id": "GO:0000981",
  "gene_name": "Cone-rod homeobox protein",
  "gene_symbol": "CRX"
}